{
  "term_id": "UNKNOWN:0001",
  "gene_name": "PTEN upstream open reading frame MP31",
  "gene_symbol": "C0HLV8",
  "gene": "UniProtKB:C0HLV8",
  "term_label": "Unknown molecular function"
}